{
  "gene": "UniProtKB:P0DMW4",
  "gene_name": "Small integral membrane protein 10-like protein 2A",
  "gene_symbol": "SMIM10L2A",
  "term_id": "UNKNOWN:0002",
  "term_label": "Unknown biological process"
}